{
  "gene_symbol": "SHROOM2",
  "term_id": "GO:0016324",
  "term_label": "apical plasma membrane",
  "gene_name": "Protein Shroom2",
  "gene": "UniProtKB:Q13796"
}